aminoglycoside N-acetyltransferase activity [GO:0034069] (molecular function) Also known as: kanamycin acetyltransferase activity Relationships: is a type of N-acetyltransferase activity [GO:0008080] Definition: Catalysis of the reaction: acetyl-CoA + aminoglycoside = CoA + N-acetylaminoglycoside. Sources: GOC:cb Subtypes: aminoglycoside 3-N-acetyltransferase activity [GO:0046353], aminoglycoside 6'-N-acetyltransferase activity [GO:0047663], aminoglycoside 2'-N-acetyltransferase activity [GO:0047921]